regulation of cellular extravasation [GO:0002691] (biological process) Definition: Any process that modulates the frequency, rate, or extent of cellular extravasation. Subtypes: negative regulation of cellular extravasation [GO:0002692], positive regulation of cellular extravasation [GO:0002693], regulation of leukocyte tethering or rolling [GO:1903236], GO:2000389, regulation of T cell extravasation [GO:2000407], GO:2000419, GO:2000437 Sources: GOC:add Relationships: is a type of GO:0002685; regulates cellular extravasation [GO:0045123]